snRNA 2'-O-ribose methylation guide activity [GO:0030563] (molecular function) Definition: Activity that provides specificity to a methylase by using base complementarity to guide site-specific 2'-O-ribose methylations to a small nuclear RNA molecule. Relationships: is_a RNA 2'-O-ribose methylation guide activity [GO:0030561]; is a type of snRNA modification guide activity [GO:0030566] Note: Note that this term describes the activity of a nucleic acid, usually RNA, gene product that interacts with other RNA molecules via base pairing; it should not be used to annotate proteins. Note that this term may be useful for annotating snoRNAs. References: PMID:11733745